{
  "term_id": "GO:0004722",
  "gene_name": "Serine_threonine-protein phosphatase PP1-alpha catalytic subunit",
  "gene": "UniProtKB:P62136",
  "gene_symbol": "PPP1CA",
  "term_label": "protein serine/threonine phosphatase activity"
}